diaphragm morphogenesis [GO:0060540] (biological process) Sources: GOC:dph Relationships: is a type of muscle organ morphogenesis [GO:0048644]; is part of diaphragm development [GO:0060539] Definition: The process in which the anatomical structures of the diaphragm are generated and organized.